{
  "gene_name": "1-phosphatidylinositol 4,5-bisphosphate phosphodiesterase delta-1",
  "gene": "UniProtKB:P51178",
  "term_id": "UNKNOWN:0002",
  "gene_symbol": "PLCD1",
  "term_label": "Unknown biological process"
}